{
  "gene": "UniProtKB:P32121",
  "gene_symbol": "ARRB2",
  "gene_name": "Beta-arrestin-2",
  "term_id": "GO:0002031",
  "term_label": "G protein-coupled receptor internalization"
}